{
  "gene_name": "Small cell adhesion glycoprotein",
  "gene": "UniProtKB:Q0VAQ4",
  "term_label": "Unknown cellular component",
  "gene_symbol": "SMAGP",
  "term_id": "UNKNOWN:0003"
}